{
  "gene_symbol": "SCTR",
  "term_id": "GO:0005886",
  "gene_name": "Secretin receptor",
  "term_label": "plasma membrane",
  "gene": "UniProtKB:P47872"
}